{
  "gene": "UniProtKB:Q8N9A8",
  "gene_symbol": "CNEP1R1",
  "gene_name": "Nuclear envelope phosphatase-regulatory subunit 1",
  "term_label": "Unknown biological process",
  "term_id": "UNKNOWN:0002"
}